{
  "gene_symbol": "MMP14",
  "term_id": "GO:0030574",
  "gene": "UniProtKB:P50281",
  "gene_name": "Matrix metalloproteinase-14",
  "term_label": "collagen catabolic process"
}